{
  "term_label": "Unknown molecular function",
  "gene": "UniProtKB:O14957",
  "gene_symbol": "UQCR11",
  "term_id": "UNKNOWN:0001",
  "gene_name": "Cytochrome b-c1 complex subunit 10"
}